{
  "term_id": "UNKNOWN:0003",
  "term_label": "Unknown cellular component",
  "gene": "UniProtKB:Q6JHZ5",
  "gene_symbol": "Q6JHZ5",
  "gene_name": "NS5ATP13TP1"
}